{
  "term_label": "antigen binding",
  "gene_name": "Immunoglobulin lambda constant 3",
  "term_id": "GO:0003823",
  "gene": "UniProtKB:P0DOY3",
  "gene_symbol": "IGLC3"
}